{
  "gene_symbol": "MIGA1",
  "gene_name": "Mitoguardin 1",
  "gene": "UniProtKB:Q8NAN2",
  "term_id": "GO:0008053",
  "term_label": "mitochondrial fusion"
}